{
  "term_id": "UNKNOWN:0003",
  "term_label": "Unknown cellular component",
  "gene_name": "Striated muscle preferentially expressed protein kinase",
  "gene": "UniProtKB:Q15772",
  "gene_symbol": "SPEG"
}